{
  "gene": "UniProtKB:Q96EP5",
  "gene_symbol": "DAZAP1",
  "gene_name": "DAZ-associated protein 1",
  "term_id": "GO:0048026",
  "term_label": "positive regulation of mRNA splicing, via spliceosome"
}